{
  "term_label": "Unknown cellular component",
  "term_id": "UNKNOWN:0003",
  "gene": "UniProtKB:Q8WWA1",
  "gene_name": "Transmembrane protein 40",
  "gene_symbol": "TMEM40"
}